3-sulfolactaldehyde reductase activity [GO:0061596] (molecular function) Relationships: is a type of oxidoreductase activity, acting on the CH-OH group of donors, NAD or NADP as acceptor [GO:0016616] References: PMID:24463506 Sources: EC:1.1.1.373, GOC:dph Definition: Catalysis of the reaction 2,3-dihydroxypropane-1-sulfonate + NAD+ = 3-sulfolactaldehyde + NADH + H+.